{
  "term_id": "UNKNOWN:0001",
  "gene": "UniProtKB:A6NJ69",
  "gene_symbol": "IGIP",
  "term_label": "Unknown molecular function",
  "gene_name": "IgA-inducing protein homolog"
}